negative regulation of cardiac muscle tissue growth [GO:0055022] (biological process) Subtypes: GO:0060044, negative regulation of cell growth involved in cardiac muscle cell development [GO:0061052] Sources: GOC:vk Also known as: down regulation of cardiac muscle growth, down-regulation of cardiac muscle growth, downregulation of cardiac muscle growth, inhibition of cardiac muscle growth, negative regulation of heart muscle growth Relationships: is a type of regulation of cardiac muscle tissue growth [GO:0055021]; is a type of negative regulation of heart growth [GO:0061117]; negatively regulates GO:0055017 Definition: Any process that stops, prevents, or reduces the frequency, rate or extent of cardiac muscle growth.